{
  "gene": "UniProtKB:Q8TB33",
  "term_id": "UNKNOWN:0001",
  "gene_name": "Putative uncharacterized protein encoded by LINC01560",
  "term_label": "Unknown molecular function",
  "gene_symbol": "LINC01560"
}